{
  "gene_symbol": "CHAMP1",
  "term_label": "sister chromatid biorientation",
  "gene": "UniProtKB:Q96JM3",
  "gene_name": "Chromosome alignment-maintaining phosphoprotein 1",
  "term_id": "GO:0031134"
}